hepatocyte homeostasis [GO:0036333] (biological process) Definition: Any biological process involved in the maintenance of the steady-state number of hepatocytes within a population of cells. Hepatocytes are specialized epithelial cells of the liver that are organized into interconnected plates called lobules. Relationships: is a type of homeostasis of number of cells [GO:0048872] References: PMID:19878874 Sources: CL:0000182, GOC:nhn